{
  "term_label": "acetylcholine receptor activity",
  "gene": "UniProtKB:P30926",
  "term_id": "GO:0015464",
  "gene_name": "Neuronal acetylcholine receptor subunit beta-4",
  "gene_symbol": "CHRNB4"
}